{
  "term_label": "translation",
  "gene_name": "Ribosome-recycling factor, mitochondrial",
  "gene": "UniProtKB:Q96E11",
  "gene_symbol": "MRRF",
  "term_id": "GO:0006412"
}